response to etoposide [GO:1902521] (biological process) Relationships: is a type of GO:1904631 Note: Note that this term is in the subset of terms that should not be used for direct manual annotation of gene products. It was created to be used for cross-referencing by other ontologies. Direct annotations to this term may be amended during annotation QC. References: PMID:23648065 Sources: GOC:TermGenie, GOC:dw Definition: Any process that results in a change in state or activity of a cell or an organism (in terms of movement, secretion, enzyme production, gene expression, etc.) as a result of an etoposide stimulus.